{
  "gene_symbol": "SLIT3",
  "term_label": "axon guidance",
  "term_id": "GO:0007411",
  "gene": "UniProtKB:O75094",
  "gene_name": "Slit homolog 3 protein"
}